{
  "term_label": "regulation of cytosolic calcium ion concentration",
  "term_id": "GO:0051480",
  "gene": "UniProtKB:Q6YI46",
  "gene_name": "Transmembrane protein 64",
  "gene_symbol": "TMEM64"
}